{
  "term_id": "UNKNOWN:0003",
  "term_label": "Unknown cellular component",
  "gene_symbol": "DFFB",
  "gene_name": "DNA fragmentation factor subunit beta",
  "gene": "UniProtKB:O76075"
}